{
  "term_id": "GO:0005886",
  "gene": "UniProtKB:A0A584",
  "term_label": "plasma membrane",
  "gene_name": "T cell receptor beta variable 11-2",
  "gene_symbol": "TRBV11-2"
}